{
  "gene_symbol": "LITAF",
  "gene_name": "Lipopolysaccharide-induced tumor necrosis factor-alpha factor",
  "gene": "UniProtKB:Q99732",
  "term_label": "nucleus",
  "term_id": "GO:0005634"
}